5-carboxymethyl-2-hydroxymuconate delta-isomerase activity [GO:0008704] (molecular function) Relationships: is a type of intramolecular oxidoreductase activity, transposing C=C bonds [GO:0016863] Sources: EC:5.3.3.10 Also known as: 5-carboxymethyl-2-hydroxymuconate D-isomerase activity, HHDD isomerase activity, 2-hydroxyhepta-2,4-diene-1,7-dioate isomerase, 5-carboxymethyl-2-hydroxymuconate delta2,Delta4-2-oxo,Delta3-isomerase activity, 5-carboxymethyl-2-hydroxymuconic acid isomerase activity, CHM isomerase activity, hpaG-1, hpaG1 Definition: Catalysis of the reaction: 5-carboxymethyl-2-hydroxymuconate = 5-carboxy-2-oxohept-3-enedioate.